{
  "term_label": "synapse",
  "gene_name": "Adenosine receptor A1",
  "gene_symbol": "ADORA1",
  "term_id": "GO:0045202",
  "gene": "UniProtKB:P30542"
}